{
  "term_label": "calcium-dependent phospholipid binding",
  "gene_name": "Annexin A8",
  "gene": "UniProtKB:P13928",
  "gene_symbol": "ANXA8",
  "term_id": "GO:0005544"
}